{
  "term_id": "GO:0000045",
  "gene_symbol": "ATG4A",
  "gene_name": "Cysteine protease ATG4A",
  "gene": "UniProtKB:Q8WYN0",
  "term_label": "autophagosome assembly"
}